{
  "term_id": "GO:0005737",
  "gene": "UniProtKB:P47944",
  "term_label": "cytoplasm",
  "gene_symbol": "MT4",
  "gene_name": "Metallothionein-4"
}